positive regulation of chlorophyll biosynthetic process [GO:1902326] (biological process) References: PMID:23555952 Sources: GOC:TermGenie Definition: Any process that activates or increases the frequency, rate or extent of chlorophyll biosynthetic process. Relationships: is_a regulation of chlorophyll biosynthetic process [GO:0010380]; is a type of GO:1901465; positively regulates chlorophyll biosynthetic process [GO:0015995] Also known as: positive regulation of chlorophyll anabolism, positive regulation of chlorophyll biosynthesis, positive regulation of chlorophyll formation, positive regulation of chlorophyll synthesis, up regulation of chlorophyll anabolism, up regulation of chlorophyll biosynthesis, up regulation of chlorophyll biosynthetic process, up regulation of chlorophyll formation, up regulation of chlorophyll synthesis, up-regulation of chlorophyll anabolism, up-regulation of chlorophyll biosynthesis, up-regulation of chlorophyll biosynthetic process, up-regulation of chlorophyll formation, up-regulation of chlorophyll synthesis, upregulation of chlorophyll anabolism, upregulation of chlorophyll biosynthesis, upregulation of chlorophyll biosynthetic process, upregulation of chlorophyll formation, upregulation of chlorophyll synthesis, activation of chlorophyll anabolism, activation of chlorophyll biosynthesis, activation of chlorophyll biosynthetic process, activation of chlorophyll formation, activation of chlorophyll synthesis